histamine secretion by platelet [GO:0002555] (biological process) Definition: The regulated release of histamine by a platelet or group of platelets. References: PMID:9117517 Sources: GOC:add Relationships: is a type of GO:0002441; is a type of establishment of localization in cell [GO:0051649]; is_a exocytic process [GO:0140029]; is part of GO:0002576